{
  "gene_name": "Serine_threonine-protein phosphatase 2A regulatory subunit B'' subunit gamma",
  "gene": "UniProtKB:Q969Q6",
  "gene_symbol": "PPP2R3C",
  "term_label": "centrosome",
  "term_id": "GO:0005813"
}